{
  "gene_name": "RE1-silencing transcription factor",
  "term_label": "negative regulation of DNA-templated transcription",
  "term_id": "GO:0045892",
  "gene": "UniProtKB:Q13127",
  "gene_symbol": "REST"
}